T=147 icosahedral capsid [GO:0039627] (cellular component) Sources: GOC:plm, UniProtKB-KW:KW-0167 Definition: The protein coat that surrounds the infective nucleic acid in some virus particles where the subunits (capsomeres) are arranged to form an icosahedron with T=147 symmetry. T=147 icosahedral capsid is composed of 12 pentameric and 1460 hexameric capsomeres for a total of 8820 capsid proteins. Relationships: is a type of icosahedral viral capsid [GO:0019030]